{
  "gene_symbol": "ZNF385B",
  "gene_name": "Zinc finger protein 385B",
  "term_label": "Unknown molecular function",
  "gene": "UniProtKB:Q569K4",
  "term_id": "UNKNOWN:0001"
}